{
  "gene": "UniProtKB:P54257",
  "gene_symbol": "HAP1",
  "term_id": "GO:0005102",
  "gene_name": "Huntingtin-associated protein 1",
  "term_label": "signaling receptor binding"
}